{
  "gene_symbol": "NEDD1",
  "gene_name": "Protein NEDD1",
  "term_id": "GO:0005737",
  "gene": "UniProtKB:Q8NHV4",
  "term_label": "cytoplasm"
}